NADPH binding [GO:0070402] (molecular function) Sources: GOC:mah Also known as: NADP (reduced) binding, reduced NADP binding, reduced nicotinamide adenine dinucleotide phosphate binding Definition: Binding to the reduced form, NADPH, of nicotinamide-adenine dinucleotide phosphate, a coenzyme involved in many redox and biosynthetic reactions. Relationships: is a type of anion binding [GO:0043168]; is a type of GO:0050661